5,6,7,8-tetrahydrosarcinapterin biosynthetic process [GO:1901855] (biological process) Definition: The chemical reactions and pathways resulting in the formation of 5,6,7,8-tetrahydrosarcinapterin. Relationships: is a type of GO:0072351; is a type of tetrahydromethanopterin biosynthetic process [GO:2001118] Sources: GOC:TermGenie, GOC:yaf, UniPathway:UPA00069 Also known as: 5,6,7,8-tetrahydrosarcinapterin anabolism, 5,6,7,8-tetrahydrosarcinapterin biosynthesis, 5,6,7,8-tetrahydrosarcinapterin formation, 5,6,7,8-tetrahydrosarcinapterin synthesis